{
  "gene_symbol": "PHF24",
  "term_id": "GO:0005737",
  "gene": "UniProtKB:Q9UPV7",
  "term_label": "cytoplasm",
  "gene_name": "PHD finger protein 24"
}